cellular pigment accumulation [GO:0043482] (BP) Sources: GOC:jl Relationships: is a type of cellular pigmentation [GO:0033059]; is a type of pigment accumulation [GO:0043476]; is a type of GO:0051716 Subtypes: GO:0048757 Definition: The aggregation of coloring matter in a particular location in a cell, occurring in response to some external stimulus.